plasmalogen synthase activity [GO:0047159] (molecular function) Definition: Catalysis of the reaction: 1-O-(1Z-alkenyl)-sn-glycero-3-phosphocholine + an acyl-CoA = 1-O-(1Z-alkenyl)-2-acyl-sn-glycero-3-phosphocholine + CoA. Sources: RHEA:10344 Relationships: is a type of O-acyltransferase activity [GO:0008374] Also known as: 1-alkenylglycerophosphocholine O-acyltransferase activity, acyl-CoA:1-alkenylglycerophosphocholine O-acyltransferase activity